{
  "gene": "UniProtKB:O00574",
  "gene_name": "C-X-C chemokine receptor type 6",
  "gene_symbol": "CXCR6",
  "term_id": "GO:0060326",
  "term_label": "cell chemotaxis"
}